{
  "term_label": "nucleus",
  "gene_symbol": "ZNF17",
  "gene_name": "Zinc finger protein 17",
  "gene": "UniProtKB:P17021",
  "term_id": "GO:0005634"
}